{
  "term_id": "GO:0014069",
  "term_label": "postsynaptic density",
  "gene_name": "Sterile alpha motif domain-containing protein 14",
  "gene": "UniProtKB:Q8IZD0",
  "gene_symbol": "SAMD14"
}